{
  "gene_name": "Molybdate-anion transporter",
  "gene_symbol": "MFSD5",
  "term_id": "UNKNOWN:0002",
  "gene": "UniProtKB:Q6N075",
  "term_label": "Unknown biological process"
}